{
  "term_id": "UNKNOWN:0002",
  "gene_name": "Putative uncharacterized protein FLJ46641",
  "gene_symbol": "Q6ZR54",
  "gene": "UniProtKB:Q6ZR54",
  "term_label": "Unknown biological process"
}